{
  "gene": "UniProtKB:Q9NXW2",
  "term_label": "cellular response to misfolded protein",
  "gene_name": "DnaJ homolog subfamily B member 12",
  "term_id": "GO:0071218",
  "gene_symbol": "DNAJB12"
}